{
  "gene": "UniProtKB:P08887",
  "gene_symbol": "IL6R",
  "gene_name": "Interleukin-6 receptor subunit alpha",
  "term_label": "receptor complex",
  "term_id": "GO:0043235"
}